{
  "term_label": "plasma membrane",
  "gene_symbol": "QRFPR",
  "term_id": "GO:0005886",
  "gene_name": "Pyroglutamylated RF-amide peptide receptor",
  "gene": "UniProtKB:Q96P65"
}